negative regulation of endothelial cell development [GO:1901551] (biological process) Relationships: is a type of negative regulation of cell development [GO:0010721]; is a type of negative regulation of endothelial cell differentiation [GO:0045602]; is a type of GO:1901550; negatively regulates endothelial cell development [GO:0001885] Definition: Any process that stops, prevents or reduces the frequency, rate or extent of endothelial cell development. References: PMID:19470579 Sources: GOC:TermGenie, GOC:pr Also known as: down regulation of endothelial cell development, down-regulation of endothelial cell development, downregulation of endothelial cell development, inhibition of endothelial cell development Subtypes: negative regulation of establishment of endothelial barrier [GO:1903141]